{
  "term_label": "signal transduction",
  "gene_name": "C-type lectin domain family 12 member A",
  "gene": "UniProtKB:Q5QGZ9",
  "term_id": "GO:0007165",
  "gene_symbol": "CLEC12A"
}